primary piRNA processing [GO:0140990] (biological process) Definition: The process involved in converting precursor piRNAs into non-overlapping, contiguous primary piRNAs (approximately 24-30-nt piRNAs with a preference for a 5' uridine (U) via the endonucleolytic activity of cytosolic PIWI. This may include pre-piRNA maturation of 3' ends by trimming and 2'-O-methylation. Relationships: is a type of piRNA processing [GO:0034587] References: PMID:22907665, PMID:26166577, PMID:34469728